{
  "gene": "UniProtKB:Q9H3M7",
  "gene_symbol": "TXNIP",
  "gene_name": "Thioredoxin-interacting protein",
  "term_label": "response to oxidative stress",
  "term_id": "GO:0006979"
}